rhombomere 5 structural organization [GO:0021665] (biological process) Also known as: rhombomere 5 structural organisation Relationships: is_a rhombomere structural organization [GO:0021595]; is part of rhombomere 5 morphogenesis [GO:0021664] Definition: The process that contributes to creating the structural organization of rhombomere 5. This process pertains to the physical shaping of a rudimentary structure. Rhombomeres are transverse segments of the developing rhombencephalon. Rhombomeres are lineage restricted, express different genes from one another, and adopt different developmental fates. Rhombomeres are numbered in an anterior to posterior order. Sources: GOC:cls, GOC:dgh, GOC:dph, GOC:jid, GO_REF:0000021